virogenic stroma [GO:0039720] (CC) Definition: A nuclear viral factory formed by Baculoviruses. A vesicular structure in which virions are assembled. Also known as: VS Relationships: is a type of GO:0039715 References: PMID:13358757, PMID:1433508 Sources: VZ:1951